2,4-diaminopentanoate dehydrogenase activity [GO:0047530] (molecular function) Definition: Catalysis of the reaction: 2,4-diaminopentanoate + H2O + NAD(P)+ = 2-amino-4-oxopentanoate + NH3 + NAD(P)H + H+. Sources: EC:1.4.1.12, MetaCyc:24-DIAMINOPENTANOATE-DEHYDROGENASE-RXN Also known as: 2,4-diaminopentanoate:NAD(P)+ oxidoreductase (deaminating), 2,4-diaminopentanoic acid C4 dehydrogenase activity Relationships: is a type of oxidoreductase activity, acting on the CH-NH2 group of donors, NAD or NADP as acceptor [GO:0016639]